hypoblast development [GO:0090008] (biological process) Definition: The process whose specific outcome is the progression of the hypoblast over time, from its formation to the mature structure. The hypoblast is a tissue formed from the inner cell mass that lies beneath the epiblast. Sources: GOC:dph, GOC:sdb_2009, GOC:tb Relationships: is a type of GO:0009888